{
  "gene": "UniProtKB:Q9H1A7",
  "gene_name": "DNA-directed RNA polymerase II subunit RPB11-b2",
  "gene_symbol": "POLR2J3",
  "term_id": "GO:0005665",
  "term_label": "RNA polymerase II, core complex"
}